negative regulation of hexadecanal biosynthetic process [GO:1900903] (biological process) Definition: Any process that stops, prevents or reduces the frequency, rate or extent of hexadecanal biosynthetic process. Also known as: down regulation of hexadecanal biosynthetic process, down-regulation of hexadecanal biosynthetic process, downregulation of hexadecanal biosynthetic process, inhibition of hexadecanal anabolism, inhibition of hexadecanal biosynthesis, inhibition of hexadecanal biosynthetic process, inhibition of hexadecanal formation, inhibition of hexadecanal synthesis, inhibition of palmitaldehyde biosynthesis, inhibition of palmitaldehyde biosynthetic process, down regulation of hexadecanal anabolism, down regulation of hexadecanal biosynthesis, down regulation of hexadecanal formation, down regulation of hexadecanal synthesis, down regulation of palmitaldehyde biosynthesis, down regulation of palmitaldehyde biosynthetic process, down-regulation of hexadecanal anabolism, down-regulation of hexadecanal biosynthesis, down-regulation of hexadecanal formation, down-regulation of hexadecanal synthesis, down-regulation of palmitaldehyde biosynthesis, down-regulation of palmitaldehyde biosynthetic process, downregulation of hexadecanal anabolism, downregulation of hexadecanal biosynthesis, downregulation of hexadecanal formation, downregulation of hexadecanal synthesis, downregulation of palmitaldehyde biosynthesis, downregulation of palmitaldehyde biosynthetic process, negative regulation of hexadecanal anabolism, negative regulation of hexadecanal biosynthesis, negative regulation of hexadecanal formation, negative regulation of hexadecanal synthesis, negative regulation of palmitaldehyde biosynthesis, negative regulation of palmitaldehyde biosynthetic process Relationships: is a type of negative regulation of biosynthetic process [GO:0009890]; is_a regulation of hexadecanal biosynthetic process [GO:1900902]; negatively regulates hexadecanal biosynthetic process [GO:0006634] Sources: GOC:TermGenie, GOC:mengo_curators